{
  "gene_name": "Transducin beta-like protein 2",
  "term_id": "GO:0030968",
  "term_label": "endoplasmic reticulum unfolded protein response",
  "gene_symbol": "TBL2",
  "gene": "UniProtKB:Q9Y4P3"
}